{
  "term_label": "hair follicle morphogenesis",
  "gene_name": "Keratin, type I cytoskeletal 27",
  "term_id": "GO:0031069",
  "gene_symbol": "KRT27",
  "gene": "UniProtKB:Q7Z3Y8"
}